{
  "gene_symbol": "TYMP",
  "term_id": "GO:0009032",
  "gene_name": "Thymidine phosphorylase",
  "term_label": "thymidine phosphorylase activity",
  "gene": "UniProtKB:P19971"
}